{
  "gene": "UniProtKB:Q8TEQ0",
  "gene_name": "Sorting nexin-29",
  "term_id": "UNKNOWN:0002",
  "term_label": "Unknown biological process",
  "gene_symbol": "SNX29"
}